protein histidine kinase binding [GO:0043424] (molecular function) Also known as: histidine kinase binding, histidine-protein kinase binding, protein-histidine kinase binding Relationships: is a type of GO:0019901 Sources: GOC:jl Definition: Binding to a protein histidine kinase.